positive regulation of membrane protein ectodomain proteolysis [GO:0051044] (biological process) Also known as: up regulation of membrane protein ectodomain proteolysis, up-regulation of membrane protein ectodomain proteolysis, upregulation of membrane protein ectodomain proteolysis, activation of membrane protein ectodomain proteolysis, stimulation of membrane protein ectodomain proteolysis Relationships: is a type of positive regulation of protein catabolic process [GO:0045732]; is a type of positive regulation of proteolysis [GO:0045862]; is a type of regulation of membrane protein ectodomain proteolysis [GO:0051043]; positively regulates membrane protein ectodomain proteolysis [GO:0006509] Sources: GOC:ai Definition: Any process that activates or increases the frequency, rate or extent of membrane protein ectodomain peptidolysis.